{
  "term_id": "GO:0045604",
  "gene_symbol": "MAFF",
  "term_label": "regulation of epidermal cell differentiation",
  "gene_name": "Transcription factor MafF",
  "gene": "UniProtKB:Q9ULX9"
}